{
  "term_id": "GO:0005886",
  "gene_symbol": "HSPA8",
  "gene_name": "Heat shock cognate 71 kDa protein",
  "term_label": "plasma membrane",
  "gene": "UniProtKB:P11142"
}